{
  "term_id": "UNKNOWN:0002",
  "term_label": "Unknown biological process",
  "gene_name": "Epithelial membrane protein 3",
  "gene": "UniProtKB:P54852",
  "gene_symbol": "EMP3"
}